{
  "gene": "UniProtKB:Q6ZNE5",
  "gene_symbol": "ATG14",
  "term_label": "autophagosome membrane docking",
  "gene_name": "Beclin 1-associated autophagy-related key regulator",
  "term_id": "GO:0016240"
}